{
  "gene_name": "LHFPL tetraspan subfamily member 2 protein",
  "gene": "UniProtKB:Q6ZUX7",
  "term_label": "Unknown biological process",
  "gene_symbol": "LHFPL2",
  "term_id": "UNKNOWN:0002"
}